{
  "gene": "UniProtKB:P22749",
  "gene_name": "Granulysin",
  "term_label": "defense response to bacterium",
  "term_id": "GO:0042742",
  "gene_symbol": "GNLY"
}